{
  "term_label": "actin binding",
  "gene_name": "Profilin-2",
  "gene_symbol": "PFN2",
  "gene": "UniProtKB:P35080",
  "term_id": "GO:0003779"
}